{
  "term_id": "GO:0046540",
  "gene": "UniProtKB:Q9Y333",
  "gene_symbol": "LSM2",
  "gene_name": "U6 snRNA-associated Sm-like protein LSm2",
  "term_label": "U4/U6 x U5 tri-snRNP complex"
}